hexose biosynthetic process [GO:0019319] (biological process) Subtypes: gluconeogenesis [GO:0006094], rhamnose biosynthetic process [GO:0019300], mannose biosynthetic process [GO:0019307], D-allose biosynthetic process [GO:0019315], GO:0042353, L-sorbose biosynthetic process [GO:0042849], GO:0046369, fructose biosynthetic process [GO:0046370] Sources: ISBN:0198506732 Relationships: is a type of GO:0019318; is a type of monosaccharide biosynthetic process [GO:0046364] Also known as: hexose anabolism, hexose biosynthesis, hexose formation, hexose synthesis Definition: The chemical reactions and pathways resulting in the formation of hexose, any monosaccharide with a chain of six carbon atoms in the molecule.